cell-matrix adhesion [GO:0007160] (biological process) Definition: The binding of a cell to the extracellular matrix via adhesion molecules. Sources: GOC:hb Subtypes: cell-matrix adhesion involved in ameboidal cell migration [GO:0003366], GO:0007161, calcium-dependent cell-matrix adhesion [GO:0016340], mesangial cell-matrix adhesion [GO:0035759], smooth muscle cell-matrix adhesion [GO:0061302], endothelial cell-matrix adhesion [GO:0090673], synaptic membrane adhesion to extracellular matrix [GO:0099561] Relationships: is a type of cell-substrate adhesion [GO:0031589] Regulation: regulated by regulation of cell-matrix adhesion [GO:0001952]; negatively regulated by negative regulation of cell-matrix adhesion [GO:0001953]; positively regulated by GO:0001954